{
  "term_id": "GO:0005764",
  "gene_symbol": "CST7",
  "gene": "UniProtKB:O76096",
  "term_label": "lysosome",
  "gene_name": "Cystatin-F"
}